cell cycle DNA replication termination [GO:1902294] (biological process) Sources: GOC:TermGenie, GOC:mtg_cell_cycle Subtypes: nuclear DNA replication termination [GO:1902317], GO:1902329 Definition: Any DNA replication termination that is involved in cell cycle DNA replication. Relationships: is a type of GO:0006274; is a type of GO:0022402; is part of cell cycle DNA replication [GO:0044786] Also known as: DNA replication termination involved in cell cycle DNA replication